{
  "gene": "UniProtKB:Q8NH04",
  "gene_name": "Olfactory receptor 2T27",
  "term_id": "GO:0004984",
  "gene_symbol": "OR2T27",
  "term_label": "olfactory receptor activity"
}